{
  "gene_name": "Putative uncharacterized protein MRGPRG-AS1",
  "term_id": "UNKNOWN:0001",
  "gene_symbol": "MRGPRG-AS1",
  "term_label": "Unknown molecular function",
  "gene": "UniProtKB:Q2M3A8"
}